{
  "term_label": "smoothened binding",
  "gene_symbol": "BBS1",
  "gene_name": "Bardet-Biedl syndrome 1 protein",
  "gene": "UniProtKB:Q8NFJ9",
  "term_id": "GO:0005119"
}